{
  "term_id": "GO:0005615",
  "gene_name": "C-C motif chemokine 14",
  "gene_symbol": "CCL14",
  "gene": "UniProtKB:Q16627",
  "term_label": "extracellular space"
}